{
  "term_label": "cytoplasm",
  "gene_name": "Prostaglandin G_H synthase 2",
  "gene": "UniProtKB:P35354",
  "gene_symbol": "PTGS2",
  "term_id": "GO:0005737"
}